{
  "gene_name": "Flt3-interacting zinc finger protein 1",
  "gene_symbol": "FIZ1",
  "term_id": "UNKNOWN:0002",
  "term_label": "Unknown biological process",
  "gene": "UniProtKB:Q96SL8"
}